pyridoxal import across plasma membrane [GO:0140204] (biological process) Sources: GOC:vw Relationships: is a type of import across plasma membrane [GO:0098739]; is a type of pyridoxal transmembrane transport [GO:1903090] Definition: The directed movement of pyridoxal from outside of a cell, across the plasma membrane and into the cytosol.